{
  "term_label": "sulfuric ester hydrolase activity",
  "gene": "UniProtKB:Q5FYB0",
  "gene_symbol": "ARSJ",
  "gene_name": "Arylsulfatase J",
  "term_id": "GO:0008484"
}